{
  "gene_symbol": "ZNF197",
  "term_id": "GO:0005634",
  "term_label": "nucleus",
  "gene": "UniProtKB:O14709",
  "gene_name": "Zinc finger protein 197"
}